peptide crotonyltransferase activity [GO:0140064] (molecular function) Subtypes: histone crotonyltransferase activity [GO:0140068] References: PMID:25818647 Also known as: protein crotonyltransferase activity Definition: Catalysis of the reaction: crotonyl-CoA + lysine in peptide = CoA + N-crotonyl-lysine-peptide. Relationships: is a type of N-acyltransferase activity [GO:0016410]